L-aspartate transmembrane export from vacuole [GO:0089703] (biological process) Relationships: is a type of vacuolar transmembrane transport [GO:0034486]; is a type of vacuolar amino acid transmembrane transport [GO:0034487]; is a type of L-aspartate transmembrane transport [GO:0070778] References: PMID:21307582 Definition: The directed movement of L-aspartate out of the vacuole, across the vacuolar membrane.